{
  "gene_symbol": "FTH1",
  "gene": "UniProtKB:P02794",
  "gene_name": "Ferritin heavy chain",
  "term_label": "ferric iron binding",
  "term_id": "GO:0008199"
}